{
  "gene": "UniProtKB:P14649",
  "term_id": "GO:0008307",
  "gene_name": "Myosin light chain 6B",
  "gene_symbol": "MYL6B",
  "term_label": "structural constituent of muscle"
}